{
  "term_id": "GO:0099560",
  "gene": "UniProtKB:P55285",
  "gene_symbol": "CDH6",
  "term_label": "synaptic membrane adhesion",
  "gene_name": "Cadherin-6"
}